{
  "gene_name": "Zinc finger protein 565",
  "gene": "UniProtKB:Q8N9K5",
  "gene_symbol": "ZNF565",
  "term_id": "GO:0006357",
  "term_label": "regulation of transcription by RNA polymerase II"
}